{
  "gene_symbol": "JMY",
  "term_id": "GO:0072332",
  "gene": "UniProtKB:Q8N9B5",
  "gene_name": "Junction-mediating and -regulatory protein",
  "term_label": "intrinsic apoptotic signaling pathway by p53 class mediator"
}